{
  "term_label": "membrane",
  "gene_symbol": "CLPTM1L",
  "term_id": "GO:0016020",
  "gene_name": "Lipid scramblase CLPTM1L",
  "gene": "UniProtKB:Q96KA5"
}